regionalization involved in semicircular canal formation [GO:0060877] (BP) Definition: The pattern specification process that results in the subdivision of the otic epithelium in space to define an area or volume in which cells will differentiate to give rise to the semicircular canals. Sources: GOC:dph, GOC:sdb_2009, GOC:tb Relationships: is a type of regionalization [GO:0003002]; is part of GO:0060876